{
  "gene": "UniProtKB:P52790",
  "term_label": "glycolytic process",
  "gene_name": "Hexokinase-3",
  "gene_symbol": "HK3",
  "term_id": "GO:0006096"
}